{
  "gene_name": "C-X-C chemokine receptor type 5",
  "gene_symbol": "CXCR5",
  "gene": "UniProtKB:P32302",
  "term_id": "GO:0006955",
  "term_label": "immune response"
}